chromosome movement towards spindle pole [GO:0051305] (biological process) Definition: The directed movement of chromosomes in the center of the spindle towards the spindle poles, mediated by the shortening of microtubules attached to the chromosomes. Sources: GOC:ai Relationships: is a type of microtubule-based movement [GO:0007018]; is a type of cell cycle process [GO:0022402]; is_a chromosome localization [GO:0050000]; is part of nuclear chromosome segregation [GO:0098813] Subtypes: mitotic chromosome movement towards spindle pole [GO:0007079], meiotic chromosome movement towards spindle pole [GO:0016344] Also known as: chromosome movement, chromosome migration to spindle pole, chromosome movement to spindle pole